ornithine aminotransferase activity [GO:0004587] (molecular function) Sources: EC:2.6.1.13 Definition: Catalysis of the reaction: a 2-oxocarboxylate + L-ornithine = an L-alpha-amino acid + L-glutamate 5-semialdehyde. Also known as: ornithine-oxo-acid aminotransferase activity, GabT, L-ornithine 5-aminotransferase activity, L-ornithine aminotransferase activity, L-ornithine:2-oxo-acid aminotransferase activity, L-ornithine:alpha-ketoglutarate delta-aminotransferase activity, OAT, ornithine 5-aminotransferase activity, ornithine delta-transaminase activity, ornithine ketoacid aminotransferase activity, ornithine transaminase activity, ornithine(lysine) transaminase activity, ornithine--2-oxoacid aminotransferase activity, ornithine--alpha-ketoglutarate aminotransferase activity, ornithine--keto acid aminotransferase activity, ornithine--keto acid transaminase activity, ornithine--ketoglutarate aminotransferase activity, ornithine--oxo acid aminotransferase activity, ornithine--oxo-acid transaminase activity, ornithine-oxo-acid transaminase activity, ornithine:alpha-oxoglutarate transaminase activity Relationships: is a type of GO:0008483